anterograde trans-synaptic signaling by nitric oxide [GO:0098940] (biological process) Definition: Cell-cell signaling from presynapse to postynapse, across the synaptic cleft, mediated by nitric oxide. Sources: GOC:dos Relationships: is a type of anterograde trans-synaptic signaling [GO:0098916]; is a type of GO:0099548